neural plate morphogenesis [GO:0001839] (biological process) Relationships: is_a morphogenesis of embryonic epithelium [GO:0016331]; is part of neural plate development [GO:0001840] Definition: The process in which the anatomical structures of the neural plate are generated and organized. The neural plate is a specialized region of columnar epithelial cells in the dorsal ectoderm that will give rise to nervous system tissue. Sources: GOC:dph, ISBN:0878932437